{
  "term_id": "GO:0005654",
  "gene_name": "Mesoderm induction early response protein 1",
  "gene_symbol": "MIER1",
  "gene": "UniProtKB:Q8N108",
  "term_label": "nucleoplasm"
}